{
  "gene_name": "Aquaporin-5",
  "gene_symbol": "AQP5",
  "term_id": "GO:0006833",
  "term_label": "water transport",
  "gene": "UniProtKB:P55064"
}